{
  "gene_name": "KxDL motif-containing protein 1",
  "term_id": "UNKNOWN:0001",
  "gene_symbol": "KXD1",
  "term_label": "Unknown molecular function",
  "gene": "UniProtKB:Q9BQD3"
}